positive regulation of actin filament polymerization [GO:0030838] (biological process) Note: Note that this term was split from 'positive regulation of actin polymerization and/or depolymerization ; GO:0045758' (sibling term 'positive regulation of actin depolymerization ; GO:0030836'). Definition: Any process that activates or increases the frequency, rate or extent of actin polymerization. Subtypes: negative regulation of barbed-end actin filament capping [GO:2000813] Sources: GOC:mah Also known as: positive regulation of actin polymerization and/or depolymerization, positive regulation of actin polymerization, up regulation of actin filament polymerization, up-regulation of actin filament polymerization, upregulation of actin filament polymerization, activation of actin filament polymerization, stimulation of actin filament polymerization Relationships: is a type of regulation of actin filament polymerization [GO:0030833]; is a type of GO:0032273; is a type of GO:0051495; is a type of GO:1902905; positively regulates actin filament polymerization [GO:0030041]